antifungal humoral response [GO:0019732] (biological process) Definition: An immune response against a fungus mediated through a body fluid. An example of this process is the antifungal humoral response in Drosophila melanogaster. Sources: GOC:go_curators, GOC:mtg_sensu Relationships: is a type of GO:0019730; is a type of defense response to fungus [GO:0050832]